{
  "term_label": "plasma membrane",
  "gene": "UniProtKB:Q5SSG8",
  "term_id": "GO:0005886",
  "gene_symbol": "MUC21",
  "gene_name": "Mucin-21"
}